{
  "gene": "UniProtKB:P30837",
  "term_label": "aldehyde dehydrogenase (NAD+) activity",
  "gene_symbol": "ALDH1B1",
  "term_id": "GO:0004029",
  "gene_name": "Aldehyde dehydrogenase X, mitochondrial"
}